{
  "gene_name": "Tryptase gamma",
  "gene_symbol": "TPSG1",
  "term_label": "serine-type endopeptidase activity",
  "term_id": "GO:0004252",
  "gene": "UniProtKB:Q9NRR2"
}